{
  "term_id": "GO:0003677",
  "gene_name": "Jerky protein homolog",
  "gene": "UniProtKB:O75564",
  "term_label": "DNA binding",
  "gene_symbol": "JRK"
}